{
  "term_label": "plasma membrane",
  "gene_symbol": "HBEGF",
  "term_id": "GO:0005886",
  "gene_name": "Proheparin-binding EGF-like growth factor",
  "gene": "UniProtKB:Q99075"
}